{
  "gene_symbol": "IFTAP",
  "term_id": "GO:0005829",
  "term_label": "cytosol",
  "gene_name": "Intraflagellar transport-associated protein",
  "gene": "UniProtKB:Q86VG3"
}